{
  "gene": "UniProtKB:Q9H081",
  "gene_symbol": "MIS12",
  "gene_name": "Protein MIS12 homolog",
  "term_id": "GO:0051382",
  "term_label": "kinetochore assembly"
}